ventricular cardiac muscle cell fate commitment [GO:0060925] (biological process) Also known as: ventricular cardiomyocyte cell fate commitment, ventricular heart muscle cell fate commitment Relationships: is a type of cardiac muscle cell fate commitment [GO:0060923]; is part of ventricular cardiac muscle cell differentiation [GO:0055012] Sources: GOC:mtg_heart Definition: The commitment of cells to ventricular cardiac muscle cell fates and their capacity to differentiate into cardiac muscle cells of the ventricle. Cardiac muscle cells are striated muscle cells that are responsible for heart contraction.